negative regulation of receptor-mediated endocytosis [GO:0048261] (biological process) Sources: GOC:go_curators Also known as: down regulation of receptor mediated endocytosis, down-regulation of receptor mediated endocytosis, downregulation of receptor mediated endocytosis, negative regulation of receptor mediated endocytosis, inhibition of receptor mediated endocytosis Relationships: is a type of negative regulation of endocytosis [GO:0045806]; is_a regulation of receptor-mediated endocytosis [GO:0048259]; RO_0002212 GO:0006898 Subtypes: negative regulation of receptor internalization [GO:0002091], negative regulation of clathrin-dependent endocytosis [GO:1900186], negative regulation of receptor-mediated endocytosis involved in cholesterol transport [GO:1905601] Definition: Any process that stops, prevents, or reduces the frequency, rate or extent of receptor mediated endocytosis, the uptake of external materials by cells, utilizing receptors to ensure specificity of transport.